{
  "gene_symbol": "TINAG",
  "gene_name": "Tubulointerstitial nephritis antigen",
  "gene": "UniProtKB:Q9UJW2",
  "term_id": "UNKNOWN:0001",
  "term_label": "Unknown molecular function"
}